pre-B cell receptor expression [GO:0002330] (biological process) Relationships: is a type of cellular developmental process [GO:0048869]; is part of pre-B cell differentiation [GO:0002329] Definition: The process leading up to expression of the pre-B cell receptor on the surface of pre-B cells, starting with the recombination of an immunuglobulin heavy chain locus, including expression of the surrogate light chain, the association of the surrogate light chain with the heavy chain, and expression of the complete pre-B cell receptor on the cell surface. pre-B cell receptor expression is a key checkpoint in the transition of pro-B cell to pre-B cell. Regulation: negatively regulated by negative regulation of pre-B cell receptor expression [GO:0140646] References: PMID:15263090, PMID:22949502, PMID:9834086 Sources: GOC:add, GOC:jal